{
  "term_label": "disulfide oxidoreductase activity",
  "gene_symbol": "TMX4",
  "gene_name": "Thioredoxin-related transmembrane protein 4",
  "term_id": "GO:0015036",
  "gene": "UniProtKB:Q9H1E5"
}